{
  "gene": "UniProtKB:O95498",
  "term_label": "pantothenate metabolic process",
  "gene_symbol": "VNN2",
  "term_id": "GO:0015939",
  "gene_name": "Pantetheine hydrolase VNN2"
}